{
  "term_id": "GO:0005789",
  "gene_name": "Protein O-mannosyl-transferase TMTC2",
  "term_label": "endoplasmic reticulum membrane",
  "gene": "UniProtKB:Q8N394",
  "gene_symbol": "TMTC2"
}